{
  "gene_name": "Zinc finger protein 142",
  "gene_symbol": "ZNF142",
  "term_id": "GO:0000977",
  "term_label": "RNA polymerase II transcription regulatory region sequence-specific DNA binding",
  "gene": "UniProtKB:P52746"
}